{
  "gene": "UniProtKB:Q8IXB3",
  "term_id": "UNKNOWN:0001",
  "gene_symbol": "TRARG1",
  "term_label": "Unknown molecular function",
  "gene_name": "Trafficking regulator of GLUT4 1"
}